positive regulation of aggrephagy [GO:1905337] (biological process) Also known as: up regulation of aggrephagy, up-regulation of aggrephagy, upregulation of aggrephagy, activation of aggrephagy Relationships: is a type of positive regulation of macroautophagy [GO:0016239]; is a type of regulation of aggrephagy [GO:1905335]; positively regulates aggrephagy [GO:0035973] Definition: Any process that activates or increases the frequency, rate or extent of aggrephagy. References: PMID:25686248 Sources: GOC:PARL, GOC:TermGenie, GOC:pad, GO_REF:0000058